circumnutation [GO:0010031] (biological process) Relationships: is a type of multicellular organismal movement [GO:0050879] Definition: The organismal movement by which the tip of a plant organ follows a spiral pattern as a consequence of growth. Sources: GOC:mtg_MIT_16mar07, ISBN:0192801023